{
  "gene_symbol": "SSR4",
  "term_label": "Unknown molecular function",
  "gene": "UniProtKB:P51571",
  "term_id": "UNKNOWN:0001",
  "gene_name": "Translocon-associated protein subunit delta"
}